{
  "gene_symbol": "FOXD4",
  "term_id": "GO:0030154",
  "gene_name": "Forkhead box protein D4",
  "gene": "UniProtKB:Q12950",
  "term_label": "cell differentiation"
}